{
  "gene_name": "Cysteine protease ATG4C",
  "gene_symbol": "ATG4C",
  "gene": "UniProtKB:Q96DT6",
  "term_id": "GO:0005737",
  "term_label": "cytoplasm"
}